scab formation [GO:0035314] (biological process) Relationships: is_a multicellular organismal process [GO:0032501]; BFO_0000050 wound healing [GO:0042060] References: PMID:15269788 Sources: GOC:bf Definition: Formation of hardened covering (a scab) at a wound site. The scab has multiple functions including limiting blood loss, providing structural stability to the wound and guarding against infection.